regulation of inhibitory synapse assembly [GO:1905702] (biological process) Relationships: is a type of regulation of synapse assembly [GO:0051963]; regulates inhibitory synapse assembly [GO:1904862] Definition: Any process that modulates the frequency, rate or extent of inhibitory synapse assembly. References: PMID:27779093 Sources: GOC:TermGenie, GO_REF:0000058 Subtypes: negative regulation of inhibitory synapse assembly [GO:1905703], positive regulation of inhibitory synapse assembly [GO:1905704] Also known as: regulation of inhibitory synapse formation